{
  "gene_symbol": "TMEM187",
  "term_id": "UNKNOWN:0001",
  "gene_name": "Transmembrane protein 187",
  "term_label": "Unknown molecular function",
  "gene": "UniProtKB:Q14656"
}